{
  "term_label": "histone deacetylase complex",
  "term_id": "GO:0000118",
  "gene": "UniProtKB:Q9UQL6",
  "gene_symbol": "HDAC5",
  "gene_name": "Histone deacetylase 5"
}